{
  "gene_symbol": "PMS2P5",
  "term_id": "UNKNOWN:0003",
  "gene_name": "Postmeiotic segregation increased 2-like protein 5",
  "term_label": "Unknown cellular component",
  "gene": "UniProtKB:A8MQ11"
}